positive regulation of platelet formation [GO:1905221] (biological process) Definition: Any process that activates or increases the frequency, rate or extent of platelet formation. Relationships: is a type of positive regulation of cell morphogenesis [GO:0010770]; is a type of positive regulation of myeloid cell differentiation [GO:0045639]; is a type of regulation of platelet formation [GO:1905219]; positively regulates platelet formation [GO:0030220] References: PMID:10606160 Sources: GOC:TermGenie, GO_REF:0000058 Also known as: positive regulation of platelet extrusion, up regulation of platelet extrusion, up regulation of platelet formation, up-regulation of platelet extrusion, up-regulation of platelet formation, upregulation of platelet extrusion, upregulation of platelet formation, activation of platelet extrusion, activation of platelet formation